{
  "term_label": "intracellular zinc ion homeostasis",
  "gene": "UniProtKB:P80297",
  "gene_name": "Metallothionein-1X",
  "term_id": "GO:0006882",
  "gene_symbol": "MT1X"
}